{
  "term_label": "cytoplasmic side of plasma membrane",
  "gene_symbol": "RGS13",
  "gene": "UniProtKB:O14921",
  "gene_name": "Regulator of G-protein signaling 13",
  "term_id": "GO:0009898"
}